oxytocin production [GO:0036162] (biological process) Definition: The appearance of oxytocin, a cyclic nonapeptide hormone with amino acid sequence CYIQNCPLG, due to biosynthesis or secretion following a cellular stimulus, resulting in an increase in its intracellular or extracellular levels. Oxytocin is the principal uterine-contracting and milk-ejecting hormone of the posterior pituitary, and together with the neuropeptide vasopressin, is believed to influence social cognition and behavior. It also acts as a neurotransmitter in the brain. Sources: GOC:cjm, Wikipedia:Oxytocin Also known as: oxytocin biosynthesis, oxytocin secretion Note: Note that this term is intended for use when a gene product is seen to cause apparent increases in intracellular or extracellular oxytocin levels, without specific regard as to whether the increase is due to increased biosynthesis, increased secretion of preexisting oxytocin molecules, or increased conversion from precursor molecules. Relationships: is a type of gene expression [GO:0010467]; has part peptide hormone secretion [GO:0030072] Regulation: regulated by regulation of oxytocin production [GO:0140667]; positively regulated by positive regulation of oxytocin production [GO:0140668]; RO_0002212 by GO:0140669